{
  "gene_name": "Protein TESPA1",
  "term_id": "UNKNOWN:0001",
  "gene_symbol": "TESPA1",
  "gene": "UniProtKB:A2RU30",
  "term_label": "Unknown molecular function"
}